{
  "gene_name": "Homeobox protein EMX1",
  "gene_symbol": "EMX1",
  "term_id": "GO:0000981",
  "term_label": "DNA-binding transcription factor activity, RNA polymerase II-specific",
  "gene": "UniProtKB:Q04741"
}